blood circulation [GO:0008015] (biological process) Regulation: regulated by regulation of blood circulation [GO:1903522]; negatively regulated by GO:1903523; positively regulated by positive regulation of blood circulation [GO:1903524] Also known as: hemolymph circulation Relationships: is a type of circulatory system process [GO:0003013] Definition: The flow of blood through the body of an animal, enabling the transport of nutrients to the tissues and the removal of waste products. Sources: GOC:mtg_heart, ISBN:0192800825 Subtypes: cerebral blood circulation [GO:0120275], GO:1990768